{
  "gene_name": "Delta-sarcoglycan",
  "term_label": "sarcoglycan complex",
  "gene_symbol": "SGCD",
  "gene": "UniProtKB:Q92629",
  "term_id": "GO:0016012"
}